adipose tissue development [GO:0060612] (BP) Regulation: RO_0002211 by regulation of adipose tissue development [GO:1904177]; negatively regulated by GO:1904178; positively regulated by positive regulation of adipose tissue development [GO:1904179] Relationships: is a type of connective tissue development [GO:0061448]; is part of animal organ development [GO:0048513] Definition: The process whose specific outcome is the progression of adipose tissue over time, from its formation to the mature structure. Adipose tissue is specialized tissue that is used to store fat. Sources: GOC:dph Also known as: adipogenesis Subtypes: mammary gland fat development [GO:0060611], GO:0060613